{
  "term_id": "GO:0001640",
  "term_label": "adenylate cyclase inhibiting G protein-coupled glutamate receptor activity",
  "gene_symbol": "GRM6",
  "gene": "UniProtKB:O15303",
  "gene_name": "Metabotropic glutamate receptor 6"
}